{
  "gene_name": "Rho guanine nucleotide exchange factor 10-like protein",
  "term_id": "GO:0030036",
  "term_label": "actin cytoskeleton organization",
  "gene": "UniProtKB:Q9HCE6",
  "gene_symbol": "ARHGEF10L"
}